{
  "gene_symbol": "AOC2",
  "term_id": "GO:0009308",
  "term_label": "amine metabolic process",
  "gene": "UniProtKB:O75106",
  "gene_name": "Retina-specific copper amine oxidase"
}